spheroidene catabolic process [GO:1901179] (biological process) Sources: GOC:TermGenie, GOC:yaf, UniPathway:UPA00683 Definition: The chemical reactions and pathways resulting in the breakdown of spheroidene. Relationships: is a type of GO:0016124; is a type of ether catabolic process [GO:1901502] Also known as: spheroidene breakdown, spheroidene catabolism, spheroidene degradation